autolysis [GO:0001896] (biological process) Definition: A programmed cell death process observed in bacteria and filamentous fungi and leading to spontaneous death by lysis. Examples are lysis of the mother cell during sporulation of Bacillus subtilis and self-degradation of fungal cells in Aspergillus nidulans. Autolysis is also involved in bacterial biofilm formation. Relationships: is a type of programmed cell death [GO:0012501] References: PMID:10974124, PMID:19286987, PMID:26811896 Sources: GOC:add, GOC:jh2, GOC:mtg_apoptosis